{
  "gene": "UniProtKB:P59923",
  "term_label": "negative regulation of gene expression via chromosomal CpG island methylation",
  "gene_symbol": "ZNF445",
  "term_id": "GO:0044027",
  "gene_name": "Zinc finger protein 445"
}